{
  "gene_name": "Natural resistance-associated macrophage protein 1",
  "gene": "UniProtKB:P49279",
  "term_label": "metal cation:proton antiporter activity",
  "gene_symbol": "SLC11A1",
  "term_id": "GO:0051139"
}